{
  "gene_symbol": "WDR74",
  "gene_name": "WD repeat-containing protein 74",
  "term_id": "GO:0042273",
  "term_label": "ribosomal large subunit biogenesis",
  "gene": "UniProtKB:Q6RFH5"
}